{
  "gene_symbol": "POU2F2",
  "gene": "UniProtKB:P09086",
  "term_id": "GO:0006357",
  "term_label": "regulation of transcription by RNA polymerase II",
  "gene_name": "POU domain, class 2, transcription factor 2"
}